{
  "gene_name": "Isoaspartyl peptidase_L-asparaginase",
  "term_label": "asparaginase activity",
  "term_id": "GO:0004067",
  "gene_symbol": "ASRGL1",
  "gene": "UniProtKB:Q7L266"
}